spliceosomal complex assembly [GO:0000245] (biological process) Definition: The aggregation, arrangement and bonding together of a spliceosomal complex, a ribonucleoprotein apparatus that catalyzes nuclear mRNA splicing via transesterification reactions. Also known as: spliceosome assembly References: PMID:9476892 Relationships: is a type of protein-RNA complex assembly [GO:0022618]; is part of mRNA splicing, via spliceosome [GO:0000398] Subtypes: U2-type prespliceosome assembly [GO:1903241]